{
  "gene_symbol": "STXBP5L",
  "gene": "UniProtKB:Q9Y2K9",
  "gene_name": "Syntaxin-binding protein 5-like",
  "term_id": "GO:0006893",
  "term_label": "Golgi to plasma membrane transport"
}